{
  "gene_symbol": "OR52H1",
  "gene": "UniProtKB:Q8NGJ2",
  "term_id": "GO:0004984",
  "term_label": "olfactory receptor activity",
  "gene_name": "Olfactory receptor 52H1"
}